{
  "term_id": "GO:0051321",
  "gene_symbol": "CDCA2",
  "gene_name": "Cell division cycle-associated protein 2",
  "gene": "UniProtKB:Q69YH5",
  "term_label": "meiotic cell cycle"
}